{
  "gene": "UniProtKB:P22914",
  "gene_symbol": "CRYGS",
  "term_id": "GO:0007601",
  "term_label": "visual perception",
  "gene_name": "Gamma-crystallin S"
}